{
  "term_label": "regulation of neuronal synaptic plasticity",
  "gene_symbol": "SYP",
  "gene": "UniProtKB:P08247",
  "gene_name": "Synaptophysin",
  "term_id": "GO:0048168"
}